{
  "gene": "UniProtKB:Q8N0Z2",
  "term_id": "GO:0045944",
  "gene_name": "Actin-binding Rho-activating protein",
  "term_label": "positive regulation of transcription by RNA polymerase II",
  "gene_symbol": "ABRA"
}